{
  "term_label": "nucleus",
  "gene_symbol": "LGALS9C",
  "gene_name": "Galectin-9C",
  "gene": "UniProtKB:Q6DKI2",
  "term_id": "GO:0005634"
}